{
  "gene": "UniProtKB:Q17RR3",
  "term_label": "Unknown cellular component",
  "gene_symbol": "PNLIPRP3",
  "gene_name": "Pancreatic lipase-related protein 3",
  "term_id": "UNKNOWN:0003"
}